7-deoxyloganin 7-hydroxylase activity [GO:0050595] (MF) Definition: Catalysis of the reaction: 7-deoxyloganin + O2 + reduced [NADPH-hemoprotein reductase] = H+ + H2O + loganin + oxidized [NADPH-hemoprotein reductase]. References: PMID:11524113 Sources: RHEA:11452 Relationships: is a type of oxidoreductase activity, acting on paired donors, with incorporation or reduction of molecular oxygen, reduced flavin or flavoprotein as one donor, and incorporation of one atom of oxygen [GO:0016712]